sphingosine N-acyltransferase activity [GO:0050291] (molecular function) Definition: Catalysis of the reaction: acyl-CoA + sphingosine = CoA + N-acylsphingosine. Also known as: ceramide synthase activity, dihydroceramide synthase activity, acyl-CoA:sphingosine N-acyltransferase activity, ceramide synthetase activity, sphingosine acyltransferase activity Relationships: is a type of N-acyltransferase activity [GO:0016410] References: PMID:12069845 Sources: EC:2.3.1.24, MetaCyc:SPHINGOSINE-N-ACYLTRANSFERASE-RXN